{
  "gene": "UniProtKB:P0DN77",
  "term_id": "GO:0007602",
  "term_label": "phototransduction",
  "gene_symbol": "OPN1MW2",
  "gene_name": "Medium-wave-sensitive opsin 2"
}